negative regulation of butyryl-CoA catabolic process to butyrate [GO:1900501] (BP) Sources: GOC:TermGenie, GOC:mengo_curators Also known as: down regulation of butyryl-CoA catabolic process to butyrate, down regulation of butyryl-CoA catabolism to butyrate, down-regulation of butyryl-CoA catabolic process to butyrate, down-regulation of butyryl-CoA catabolism to butyrate, downregulation of butyryl-CoA catabolic process to butyrate, downregulation of butyryl-CoA catabolism to butyrate, inhibition of butyryl-CoA catabolism to butyrate, negative regulation of butyryl-CoA catabolism to butyrate, inhibition of butyryl-CoA catabolic process to butyrate Relationships: is a type of negative regulation of amide metabolic process [GO:0034249]; is a type of GO:0045717; is a type of negative regulation of nucleobase-containing compound metabolic process [GO:0045934]; is a type of GO:0045936; is a type of GO:0050995; is a type of regulation of butyryl-CoA catabolic process to butyrate [GO:1900500]; negatively regulates butyryl-CoA catabolic process to butyrate [GO:0044581] Definition: Any process that stops, prevents or reduces the frequency, rate or extent of butyryl-CoA catabolic process to butyrate.